{
  "gene_name": "Neurotrophin-3",
  "term_label": "neuron projection morphogenesis",
  "gene_symbol": "NTF3",
  "term_id": "GO:0048812",
  "gene": "UniProtKB:P20783"
}